{
  "gene": "UniProtKB:Q9UF47",
  "term_id": "UNKNOWN:0002",
  "term_label": "Unknown biological process",
  "gene_name": "DnaJ homolog subfamily C member 5B",
  "gene_symbol": "DNAJC5B"
}